localization within membrane [GO:0051668] (BP) Definition: Any process in which a substance or cellular entity, such as a protein complex or organelle, is transported to, and/or maintained in, a specific location within a membrane. Sources: GOC:ai Also known as: establishment and maintenance of localization in membrane, establishment and maintenance of position in membrane, localisation within membrane, localization to membrane, positioning within membrane Relationships: is a type of cellular localization [GO:0051641] Subtypes: lipoprotein localization to membrane [GO:0044873], GO:0051664, membrane raft localization [GO:0051665], protein localization to membrane [GO:0072657], establishment of protein localization to membrane [GO:0090150], vesicle-mediated transport to the plasma membrane [GO:0098876], receptor diffusion trapping [GO:0098953], GO:0140043, GO:0140334, ganglioside GM1 transport to membrane [GO:1905572]